{
  "gene_symbol": "GCK",
  "term_label": "cytosol",
  "gene_name": "Hexokinase-4",
  "term_id": "GO:0005829",
  "gene": "UniProtKB:P35557"
}